{
  "gene": "UniProtKB:Q9HBL0",
  "term_label": "focal adhesion",
  "gene_symbol": "TNS1",
  "term_id": "GO:0005925",
  "gene_name": "Tensin-1"
}